{
  "gene": "UniProtKB:Q9P0J0",
  "gene_symbol": "NDUFA13",
  "gene_name": "NADH dehydrogenase [ubiquinone] 1 alpha subcomplex subunit 13",
  "term_id": "GO:0045271",
  "term_label": "respiratory chain complex I"
}